{
  "gene": "UniProtKB:Q06124",
  "gene_symbol": "PTPN11",
  "gene_name": "Tyrosine-protein phosphatase non-receptor type 11",
  "term_label": "non-membrane spanning protein tyrosine phosphatase activity",
  "term_id": "GO:0004726"
}